{
  "term_label": "AMPA glutamate receptor complex",
  "gene_name": "Glutamate receptor 1",
  "gene_symbol": "GRIA1",
  "gene": "UniProtKB:P42261",
  "term_id": "GO:0032281"
}